{
  "term_label": "olfactory receptor activity",
  "gene": "UniProtKB:Q8NG97",
  "gene_symbol": "OR2Z1",
  "gene_name": "Olfactory receptor 2Z1",
  "term_id": "GO:0004984"
}